{
  "gene_symbol": "TYW3",
  "gene": "UniProtKB:Q6IPR3",
  "gene_name": "tRNA wybutosine-synthesizing protein 3 homolog",
  "term_label": "tRNA methyltransferase activity",
  "term_id": "GO:0008175"
}